indole-3-acetate carboxyl methyltransferase activity [GO:0103007] (MF) Sources: EC:2.1.1.278, GOC:pz Relationships: is a type of GO:0008168 Definition: Catalysis of the reaction: indole-3-acetate + S-adenosyl-L-methionine = methyl (indol-3-yl)acetate + S-adenosyl-L-homocysteine.